homomeric SMAD protein complex [GO:0071142] (cellular component) Relationships: is a type of GO:0071141; is part of cytoplasm [GO:0005737] Definition: A protein complex composed of a single type of SMAD family proteins. In the absence of Smad4, phosphorylation of R-SMADs results in their homotrimerization. However, these complexes do not appear to import into the nucleus and are assumed to be transcriptionally inactive. Also known as: SMAD1 homotrimer complex, SMAD1 protein complex, SMAD2 homotrimer complex, SMAD2 protein complex, SMAD3 homotrimer complex, SMAD3 protein complex References: PMID:11779505, PMID:16322555, PMID:9670020 Sources: GOC:bhm, GOC:mah